{
  "gene": "UniProtKB:O43795",
  "gene_symbol": "MYO1B",
  "gene_name": "Unconventional myosin-Ib",
  "term_label": "endocytosis",
  "term_id": "GO:0006897"
}